regulation of pinocytosis [GO:0048548] (biological process) Relationships: is a type of regulation of endocytosis [GO:0030100]; RO_0002211 pinocytosis [GO:0006907] Definition: Any process that modulates the frequency, rate or extent of pinocytosis. Pinocytosis is the process in which cells take in liquid material from their external environment; literally 'cell drinking'. Liquid is enclosed in vesicles, formed by invagination of the plasma membrane. These vesicles then move into the cell and pass their contents to endosomes. Subtypes: positive regulation of pinocytosis [GO:0048549], negative regulation of pinocytosis [GO:0048550], regulation of macropinocytosis [GO:1905301] Sources: GOC:go_curators